{
  "term_id": "GO:0005737",
  "gene": "UniProtKB:P78330",
  "gene_symbol": "PSPH",
  "term_label": "cytoplasm",
  "gene_name": "Phosphoserine phosphatase"
}